{
  "term_id": "UNKNOWN:0003",
  "gene": "UniProtKB:Q86YQ2",
  "gene_symbol": "BPIFA4P",
  "term_label": "Unknown cellular component",
  "gene_name": "Putative BPIFA4P protein"
}